{
  "term_label": "EMC complex",
  "term_id": "GO:0072546",
  "gene_symbol": "EMC4",
  "gene_name": "ER membrane protein complex subunit 4",
  "gene": "UniProtKB:Q5J8M3"
}